{
  "gene_name": "Peptidyl-tRNA hydrolase 2, mitochondrial",
  "gene": "UniProtKB:Q9Y3E5",
  "term_label": "negative regulation of anoikis",
  "gene_symbol": "PTRH2",
  "term_id": "GO:2000811"
}